autophagosome [GO:0005776] (cellular component) References: PMID:11099404 Sources: GOC:autophagy, ISBN:0198547684 Relationships: is a type of vacuole [GO:0005773] Also known as: autophagic vacuole, initial autophagic vacuole Definition: A double-membrane-bounded compartment that engulfs endogenous cellular material as well as invading microorganisms to target them to the lytic vacuole/lysosome for degradation as part of macroautophagy. Subtypes: GO:0044753